neural fold hinge point formation [GO:0021504] (biological process) Definition: The formation of the median and lateral hinge points in the neural folds. These are created by apical constriction and basal expansion of the underlying neural cells. The median hinge point extends for the entire length of the neural tube, and the lateral hinge points do not form in the spinal cord region of the neural tube. References: PMID:13679871, PMID:15806586 Sources: GOC:cls, GOC:dgh, GOC:dph, GOC:jid, GO_REF:0000021 Also known as: neural fold furrowing Relationships: is a type of anatomical structure formation involved in morphogenesis [GO:0048646]; is part of neural fold bending [GO:0021503]